{
  "term_id": "UNKNOWN:0001",
  "gene": "UniProtKB:Q6P5S2",
  "gene_name": "Protein LEG1 homolog",
  "gene_symbol": "LEG1",
  "term_label": "Unknown molecular function"
}